{
  "term_label": "Unknown cellular component",
  "gene": "UniProtKB:Q8N8E3",
  "gene_symbol": "CEP112",
  "gene_name": "Centrosomal protein of 112 kDa",
  "term_id": "UNKNOWN:0003"
}